{
  "term_id": "GO:0019814",
  "gene_name": "Immunoglobulin lambda variable 5-39",
  "gene_symbol": "IGLV5-39",
  "term_label": "immunoglobulin complex",
  "gene": "UniProtKB:A0A0G2JS06"
}